EMILIN complex [GO:1990971] (cellular component) Definition: Glycoprotein complex of the C1q/TNF superfamily found in the extracellular matrix (ECM) where it is an important component of the elastic fiber system. A homotrimer that will combine to form supramolecular EMILIN structures. References: PMID:10821830 Sources: GOC:bhm Also known as: EMILIN-1 complex, EMILIN-2 complex, Elastic microfibrillar interface 1 complex, Elastic microfibrillar interface 2 complex Note: An example of this is EMILIN-1 in human (Q9Y6C2) in PMID:10821830 (inferred from direct assay). Relationships: is a type of protein complex involved in cell-matrix adhesion [GO:0098637]; is part of extracellular matrix [GO:0031012]